{
  "term_id": "GO:0005737",
  "gene_name": "Aquaporin-12B",
  "term_label": "cytoplasm",
  "gene_symbol": "AQP12B",
  "gene": "UniProtKB:A6NM10"
}